{
  "term_id": "GO:0071385",
  "gene_symbol": "SSTR2",
  "term_label": "cellular response to glucocorticoid stimulus",
  "gene": "UniProtKB:P30874",
  "gene_name": "Somatostatin receptor type 2"
}